{
  "gene": "UniProtKB:P35611",
  "term_id": "GO:0014069",
  "term_label": "postsynaptic density",
  "gene_symbol": "ADD1",
  "gene_name": "Alpha-adducin"
}